response to human chorionic gonadotropin [GO:0044752] (biological process) Subtypes: cellular response to human chorionic gonadotropin stimulus [GO:0044751] Also known as: response to human chorionic gonadotropin stimulus References: PMID:21325635 Definition: Any process that results in a change in state or activity of a cell or organism (in terms of movement, secretion, enzyme production, gene expression, etc.) as a result of a human chorionic gonadotropin stimulus. Relationships: is a type of GO:0034698